{
  "term_label": "focal adhesion",
  "gene": "UniProtKB:Q8N264",
  "term_id": "GO:0005925",
  "gene_name": "Rho GTPase-activating protein 24",
  "gene_symbol": "ARHGAP24"
}